{
  "gene_name": "Transcription regulator protein BACH2",
  "gene_symbol": "BACH2",
  "term_id": "GO:0000981",
  "term_label": "DNA-binding transcription factor activity, RNA polymerase II-specific",
  "gene": "UniProtKB:Q9BYV9"
}